{
  "term_id": "GO:0031012",
  "gene_symbol": "CCN5",
  "gene_name": "CCN family member 5",
  "gene": "UniProtKB:O76076",
  "term_label": "extracellular matrix"
}